{
  "gene_symbol": "NUDT14",
  "term_label": "nucleoside phosphate metabolic process",
  "gene_name": "Uridine diphosphate glucose pyrophosphatase NUDT14",
  "term_id": "GO:0006753",
  "gene": "UniProtKB:O95848"
}